{
  "gene_symbol": "HADH",
  "gene": "UniProtKB:Q16836",
  "gene_name": "Hydroxyacyl-coenzyme A dehydrogenase, mitochondrial",
  "term_label": "fatty acid beta-oxidation",
  "term_id": "GO:0006635"
}